regulation of axonogenesis [GO:0050770] (biological process) Subtypes: regulation of axon diameter [GO:0031133], regulation of collateral sprouting [GO:0048670], GO:0050771, positive regulation of axonogenesis [GO:0050772] Relationships: is a type of regulation of neuron projection development [GO:0010975]; is a type of GO:0022603; regulates GO:0007409 Definition: Any process that modulates the frequency, rate or extent of axonogenesis, the generation of an axon, the long process of a neuron. Sources: GOC:ai